contractile vacuole tethering involved in discharge [GO:0140025] (BP) Relationships: is a type of GO:0006903; is a type of vesicle tethering involved in exocytosis [GO:0090522]; is part of contractile vacuole discharge [GO:0070177] References: PMID:22323285 Definition: The initial, indirect interaction between a contractile vacuole membrane and a site of discharge in the plasma membrane. This interaction is mediated by tethering factors (or complexes), which interact with both membranes. Interaction can occur via direct binding to membrane phospholipids or membrane proteins, or via binding to vesicle coat proteins. This process is distinct from and prior to docking and fusion. Also known as: contractile vacuole tethering to plasma membrane